acetate transmembrane transporter activity [GO:0015123] (molecular function) Subtypes: GO:0043893 Relationships: is a type of monocarboxylic acid transmembrane transporter activity [GO:0008028]; is part of acetate transmembrane transport [GO:0035433] Sources: GOC:ai Definition: Enables the transfer of acetate from one side of a membrane to the other. Acetate is the 2-carbon carboxylic acid ethanoic acid.